{
  "gene_symbol": "PLA2G2A",
  "gene_name": "Phospholipase A2, membrane associated",
  "gene": "UniProtKB:P14555",
  "term_label": "phospholipid binding",
  "term_id": "GO:0005543"
}